positive regulation of glucosylceramide catabolic process [GO:2000753] (biological process) Also known as: positive regulation of glucosylceramide breakdown, positive regulation of glucosylceramide catabolism, positive regulation of glucosylceramide degradation Sources: GOC:BHF Definition: Any process that activates or increases the frequency, rate or extent of glucosylceramide catabolic process. Relationships: is a type of positive regulation of amide metabolic process [GO:0034250]; is a type of positive regulation of lipid catabolic process [GO:0050996]; is a type of regulation of glucosylceramide catabolic process [GO:2000752]; positively regulates GO:0006680